positive regulation of convergent extension involved in rhombomere morphogenesis [GO:1904135] (biological process) References: PMID:24892953 Sources: GOC:TermGenie, GOC:dph, GO_REF:0000058 Relationships: is a type of positive regulation of convergent extension involved in gastrulation [GO:1904105]; is a type of regulation of convergent extension involved in rhombomere morphogenesis [GO:1904133]; positively regulates convergent extension involved in rhombomere morphogenesis [GO:1904125] Also known as: up regulation of convergent extension involved in rhombomere morphogenesis, up-regulation of convergent extension involved in rhombomere morphogenesis, upregulation of convergent extension involved in rhombomere morphogenesis, activation of convergent extension involved in rhombomere morphogenesis Definition: Any process that activates or increases the frequency, rate or extent of convergent extension involved in rhombomere morphogenesis.